poly(3-hydroxybutyrate) depolymerase activity [GO:0050526] (molecular function) Definition: Catalysis of the reaction: H2O + poly[(R)-3-hydroxybutanoate](n) = poly[(R)-3-hydroxybutanoate](x) + poly[(R)-3-hydroxybutanoate](n-x); x is 1-5. Sources: EC:3.1.1.75, MetaCyc:3.1.1.75-RXN Also known as: poly((R)-hydroxyalkanoic acid) depolymerase activity, poly[(R)-hydroxyalkanoic acid] depolymerase, PHB depolymerase activity, poly(3HB) depolymerase activity, poly(HA(SCL)) depolymerase activity, poly(HA) depolymerase activity, poly(HASCL) depolymerase activity, poly[(R)-3-hydroxybutyrate] hydrolase activity Relationships: is a type of carboxylic ester hydrolase activity [GO:0052689]